extracellularly ATP-gated monoatomic cation channel activity [GO:0004931] (molecular function) Definition: Enables the transmembrane transfer of a monoatomic cation by a channel that opens when ATP is bound by the channel complex or one of its constituent parts on the extracellular side of the plasma membrane. References: PMID:9755289 Sources: GOC:bf, GOC:mah Also known as: extracellularly ATP-gated cation channel activity, purinoceptor, purinoreceptor, P2X receptor Relationships: is a type of excitatory extracellular ligand-gated monoatomic ion channel activity [GO:0005231]; is a type of ATP-gated ion channel activity [GO:0035381]; is a type of ligand-gated monoatomic cation channel activity [GO:0099094] Note: Note that this term refers to an activity and not a gene product. Consider also annotating to the molecular function term 'purinergic nucleotide receptor activity ; GO:0001614'.